positive regulation of attachment of mitotic spindle microtubules to kinetochore [GO:1902425] (BP) Subtypes: positive regulation of mitotic sister chromatid biorientation [GO:0140429], positive regulation of lateral attachment of mitotic spindle microtubules to kinetochore [GO:1905116] References: PMID:22065639 Sources: GOC:TermGenie Definition: Any process that activates or increases the frequency, rate or extent of attachment of spindle microtubules to kinetochore involved in mitotic sister chromatid segregation. Also known as: positive regulation of attachment of spindle microtubules to kinetochore involved in mitosis, positive regulation of attachment of spindle microtubules to kinetochore involved in mitotic sister chromatid segregation, positive regulation of attachment of spindle microtubules to mitotic chromosome, up regulation of attachment of spindle microtubules to kinetochore involved in mitosis, up regulation of attachment of spindle microtubules to kinetochore involved in mitotic sister chromatid segregation, up regulation of attachment of spindle microtubules to mitotic chromosome, up-regulation of attachment of spindle microtubules to kinetochore involved in mitosis, up-regulation of attachment of spindle microtubules to kinetochore involved in mitotic sister chromatid segregation, up-regulation of attachment of spindle microtubules to mitotic chromosome, upregulation of attachment of spindle microtubules to kinetochore involved in mitosis, upregulation of attachment of spindle microtubules to kinetochore involved in mitotic sister chromatid segregation, upregulation of attachment of spindle microtubules to mitotic chromosome, activation of attachment of spindle microtubules to kinetochore involved in mitosis, activation of attachment of spindle microtubules to kinetochore involved in mitotic sister chromatid segregation, activation of attachment of spindle microtubules to mitotic chromosome, activation of attachment of spindle microtubules to kinetochore during mitosis, activation of mitotic bipolar attachment, positive regulation of attachment of spindle microtubules to kinetochore during mitosis, positive regulation of mitotic bipolar attachment, up regulation of attachment of spindle microtubules to kinetochore during mitosis, up regulation of mitotic bipolar attachment, up-regulation of attachment of spindle microtubules to kinetochore during mitosis, up-regulation of mitotic bipolar attachment, upregulation of attachment of spindle microtubules to kinetochore during mitosis, upregulation of mitotic bipolar attachment Relationships: is a type of positive regulation of attachment of spindle microtubules to kinetochore [GO:0051987]; is a type of regulation of attachment of mitotic spindle microtubules to kinetochore [GO:1902423]; positively regulates GO:0051315